{
  "gene_symbol": "ZNF716",
  "term_label": "DNA-binding transcription factor activity, RNA polymerase II-specific",
  "gene_name": "Zinc finger protein 716",
  "term_id": "GO:0000981",
  "gene": "UniProtKB:A6NP11"
}